{
  "gene_symbol": "COX6B2",
  "gene": "UniProtKB:Q6YFQ2",
  "term_id": "GO:0030061",
  "term_label": "mitochondrial crista",
  "gene_name": "Cytochrome c oxidase subunit 6B2"
}